{
  "gene": "UniProtKB:Q17RY0",
  "gene_name": "Cytoplasmic polyadenylation element-binding protein 4",
  "term_id": "GO:0005737",
  "gene_symbol": "CPEB4",
  "term_label": "cytoplasm"
}